{
  "term_label": "autophagosome",
  "gene_symbol": "FYCO1",
  "term_id": "GO:0005776",
  "gene_name": "FYVE and coiled-coil domain-containing protein 1",
  "gene": "UniProtKB:Q9BQS8"
}